{
  "gene": "UniProtKB:Q496Y0",
  "gene_symbol": "LONRF3",
  "gene_name": "LON peptidase N-terminal domain and RING finger protein 3",
  "term_label": "Unknown cellular component",
  "term_id": "UNKNOWN:0003"
}